{
  "gene_name": "Zinc finger protein 362",
  "term_id": "UNKNOWN:0003",
  "gene": "UniProtKB:Q5T0B9",
  "term_label": "Unknown cellular component",
  "gene_symbol": "ZNF362"
}